{
  "term_id": "GO:0031386",
  "gene_name": "Ubiquitin-like protein ISG15",
  "gene": "UniProtKB:P05161",
  "gene_symbol": "ISG15",
  "term_label": "protein tag activity"
}